{
  "gene": "UniProtKB:Q8TF21",
  "term_id": "UNKNOWN:0001",
  "gene_symbol": "ANKRD24",
  "gene_name": "Ankyrin repeat domain-containing protein 24",
  "term_label": "Unknown molecular function"
}